{
  "gene_symbol": "NCLN",
  "term_id": "UNKNOWN:0001",
  "term_label": "Unknown molecular function",
  "gene": "UniProtKB:Q969V3",
  "gene_name": "BOS complex subunit NCLN"
}